{
  "gene": "UniProtKB:Q96E22",
  "gene_name": "Dehydrodolichyl diphosphate synthase complex subunit NUS1",
  "term_id": "GO:0043048",
  "term_label": "dolichyl monophosphate biosynthetic process",
  "gene_symbol": "NUS1"
}